{
  "gene_symbol": "CD1C",
  "gene_name": "T-cell surface glycoprotein CD1c",
  "gene": "UniProtKB:P29017",
  "term_label": "positive regulation of T cell mediated cytotoxicity",
  "term_id": "GO:0001916"
}